positive regulation of B-1 B cell differentiation [GO:0001926] (biological process) Definition: Any process that activates or increases the frequency, rate or extent of B-1 B cell differentiation. Sources: GOC:add, ISBN:0781735149 Also known as: positive regulation of B-1 B lymphocyte differentiation, positive regulation of B-1 B-cell differentiation, positive regulation of B-1 B-lymphocyte differentiation, up regulation of B-1 B cell differentiation, up-regulation of B-1 B cell differentiation, upregulation of B-1 B cell differentiation, activation of B-1 B cell differentiation, stimulation of B-1 B cell differentiation, positive regulation of B-1 B cell development Note: Note that immunologists typically use the word 'development' to refer to cells of B or T cell lineages undergoing the process that GO describes as 'cell differentiation'. Relationships: is a type of regulation of B-1 B cell differentiation [GO:0001924]; is a type of positive regulation of B cell differentiation [GO:0045579]; positively regulates B-1 B cell differentiation [GO:0001923]